{
  "term_id": "GO:0005125",
  "gene": "UniProtKB:P10600",
  "gene_name": "Transforming growth factor beta-3 proprotein",
  "gene_symbol": "TGFB3",
  "term_label": "cytokine activity"
}